{
  "gene_name": "T-box transcription factor TBX6",
  "term_label": "DNA-binding transcription factor activity, RNA polymerase II-specific",
  "term_id": "GO:0000981",
  "gene": "UniProtKB:O95947",
  "gene_symbol": "TBX6"
}